{
  "gene_name": "C-C motif chemokine 22",
  "term_label": "CCR chemokine receptor binding",
  "gene": "UniProtKB:O00626",
  "term_id": "GO:0048020",
  "gene_symbol": "CCL22"
}